{
  "gene_name": "Rho GTPase-activating protein 22",
  "gene_symbol": "ARHGAP22",
  "gene": "UniProtKB:Q7Z5H3",
  "term_label": "GTPase activator activity",
  "term_id": "GO:0005096"
}